{
  "gene_name": "Histone-lysine N-methyltransferase 2C",
  "term_id": "GO:0140945",
  "term_label": "histone H3K4 monomethyltransferase activity",
  "gene_symbol": "KMT2C",
  "gene": "UniProtKB:Q8NEZ4"
}